MRF binding [GO:0043426] (MF) References: PMID:10966875 Relationships: is a type of bHLH transcription factor binding [GO:0043425] Also known as: Mrf4 binding, Myf5 binding, MyoD binding, myogenin binding Definition: Binding to Myogenic Regulatory Factor (MRF), a member of the basic Helix-Loop-Helix (bHLH) superfamily of transcription factors.